{
  "term_id": "GO:0005634",
  "gene_symbol": "ALX4",
  "gene": "UniProtKB:Q9H161",
  "gene_name": "Homeobox protein aristaless-like 4",
  "term_label": "nucleus"
}